{
  "term_id": "GO:0017174",
  "term_label": "glycine N-methyltransferase activity",
  "gene": "UniProtKB:Q14749",
  "gene_name": "Glycine N-methyltransferase",
  "gene_symbol": "GNMT"
}